{
  "term_label": "Unknown cellular component",
  "gene": "UniProtKB:P36542",
  "gene_name": "ATP synthase subunit gamma, mitochondrial",
  "gene_symbol": "ATP5F1C",
  "term_id": "UNKNOWN:0003"
}